{
  "gene": "UniProtKB:P78334",
  "term_label": "chloride transmembrane transport",
  "term_id": "GO:1902476",
  "gene_symbol": "GABRE",
  "gene_name": "Gamma-aminobutyric acid receptor subunit epsilon"
}